cellular response to oxygen-containing compound [GO:1901701] (biological process) Relationships: is a type of cellular response to chemical stimulus [GO:0070887]; is a type of GO:1901700 Subtypes: cellular response to reactive oxygen species [GO:0034614], GO:0035714, GO:0035984, cellular response to L-canavanine [GO:0036280], cellular response to sterol [GO:0036315], GO:0036346, GO:0061431, cellular response to 1-aminocyclopropane-1-carboxylic acid [GO:0071213], cellular response to lipopolysaccharide [GO:0071222], cellular response to lipoteichoic acid [GO:0071223], GO:0071224, cellular response to muramyl dipeptide [GO:0071225], cellular response to folic acid [GO:0071231], cellular response to histidine [GO:0071232], cellular response to L-leucine [GO:0071233], cellular response to phenylalanine [GO:0071234], cellular response to proline [GO:0071235], cellular response to bacteriocin [GO:0071237], cellular response to brefeldin A [GO:0071238], cellular response to streptomycin [GO:0071239], cellular response to carbon dioxide [GO:0071244], cellular response to carbon monoxide [GO:0071245], cellular response to chlorate [GO:0071246], cellular response to chromate [GO:0071247], cellular response to nitrate [GO:0071249], GO:0071250, cellular response to silicon dioxide [GO:0071251], cellular response to sulfur dioxide [GO:0071252], cellular response to tellurium ion [GO:0071293], cellular response to biotin [GO:0071296], cellular response to cobalamin [GO:0071297], cellular response to retinoic acid [GO:0071300], GO:0071302, cellular response to vitamin B6 [GO:0071304], GO:0071305, cellular response to vitamin E [GO:0071306], GO:0071311, cellular response to cocaine [GO:0071314], GO:0071318, cellular response to benzoic acid [GO:0071319], cellular response to cAMP [GO:0071320], cellular response to cGMP [GO:0071321], cellular response to carbohydrate stimulus [GO:0071322], cellular response to chitin [GO:0071323], cellular response to ether [GO:0071362], cellular response to indolebutyric acid stimulus [GO:0071366], cellular response to brassinosteroid stimulus [GO:0071367], cellular response to gibberellin stimulus [GO:0071370], GO:0071375, cellular response to prostaglandin I stimulus [GO:0071382], cellular response to estradiol stimulus [GO:0071392], cellular response to fatty acid [GO:0071398], cellular response to triglyceride [GO:0071401], cellular response to methotrexate [GO:0071414], cellular response to salicylic acid stimulus [GO:0071446], cellular response to hydroperoxide [GO:0071447], GO:0071462, GO:0071504, cellular response to mycophenolic acid [GO:0071506], cellular response to nitric oxide [GO:0071732], cellular response to catecholamine stimulus [GO:0071870], cellular response to methyl methanesulfonate [GO:0072703], cellular response to sodium dodecyl sulfate [GO:0072707], cellular response to selenite ion [GO:0072715], cellular response to actinomycin D [GO:0072717], cellular response to dithiothreitol [GO:0072721], cellular response to 4-nitroquinoline N-oxide [GO:0072725], cellular response to papulacandin B [GO:0072731], cellular response to erythromycin [GO:0072743], cellular response to antimycin A [GO:0072745], cellular response to chloramphenicol [GO:0072747], cellular response to tacrolimus [GO:0072748], cellular response to cytochalasin B [GO:0072749], cellular response to L-thialysine [GO:0072751], GO:0072753, cellular response to hesperadin [GO:0072763], cellular response to thyroxine stimulus [GO:0097069], GO:0097306, cellular response to N-acetyl-D-glucosamine [GO:0097316], cellular response to aldehyde [GO:0110096], cellular response to ketone [GO:1901655], cellular response to diethyl maleate [GO:1902112], cellular response to inositol [GO:1902141], GO:1902348, GO:1902439, cellular response to bile acid [GO:1903413], cellular response to L-arginine [GO:1903577], cellular response to arsenite(3-) [GO:1903841], GO:1903843, cellular response to bisphenol A [GO:1903926], cellular response to acrylamide [GO:1903938], cellular response to micafungin [GO:1903968], cellular response to serotonin [GO:1904015], GO:1904102, cellular response to cordycepin [GO:1904310], cellular response to kainic acid [GO:1904374], cellular response to D-galactosamine [GO:1904422], cellular response to L-dopa [GO:1904474], cellular response to tetrahydrofolate [GO:1904482], GO:1904566, GO:1904588, cellular response to glucoside [GO:1904632], cellular response to resveratrol [GO:1904639], cellular response to dinitrophenol [GO:1904642], cellular response to amyloid-beta [GO:1904646], cellular response to nitroglycerin [GO:1904843], cellular response to L-glutamine [GO:1904845], cellular response to bleomycin [GO:1904976], cellular response to acetylcholine [GO:1905145], cellular response to L-glutamate [GO:1905232], cellular response to cyclosporin A [GO:1905238], cellular response to 3,3',5-triiodo-L-thyronine [GO:1905243], cellular response to homocysteine [GO:1905375], cellular response to flavonoid [GO:1905396], cellular response to glycine [GO:1905430], cellular response to chondroitin 6'-sulfate [GO:1905440], cellular response to chondroitin 4'-sulfate [GO:1905442], cellular response to phosphatidylethanolamine [GO:1905712], GO:1905795, cellular response to pyrimidine ribonucleotide [GO:1905835] Also known as: cellular response to oxygen molecular entity Definition: Any process that results in a change in state or activity of a cell (in terms of movement, secretion, enzyme production, gene expression, etc.) as a result of an oxygen-containing compound stimulus. Sources: GOC:TermGenie, GOC:pr